{
  "term_id": "GO:0031072",
  "term_label": "heat shock protein binding",
  "gene_symbol": "CDC37L1",
  "gene": "UniProtKB:Q7L3B6",
  "gene_name": "Hsp90 co-chaperone Cdc37-like 1"
}